{
  "gene_name": "Methylmalonate-semialdehyde dehydrogenase [acylating], mitochondrial",
  "term_id": "GO:0006574",
  "gene_symbol": "ALDH6A1",
  "gene": "UniProtKB:Q02252",
  "term_label": "L-valine catabolic process"
}